cellulose microfibril [GO:0009549] (cellular component) Definition: A microfibril composed of cellulose arranged in orthogonal layers. Cellulose is a straight chain polysaccharide composed of B(14) linked glucose subunits. It is a major component of plant cell walls. Higher plant microfibrils are about 10nm in diameter and extremely long in relation to their width. The cellulose molecules are oriented parallel to the long axis of the microfibril in a paracrystalline array, which provides great tensile strength. The microfibrils are held in place by the wall matrix and their orientation is closely controlled by the cell. Relationships: is a type of cellular anatomical structure [GO:0110165]; is part of GO:0009505 Sources: GOC:jid, ISBN:0943088399